replication-born double-strand break repair via sister chromatid exchange [GO:1990414] (biological process) Relationships: is a type of double-strand break repair via homologous recombination [GO:0000724] References: PMID:12820977, PMID:16888651 Sources: GOC:rb Also known as: replication-born DSB repair by SCE Definition: The repair of a replication-born double-strand DNA break in which the DNA molecule is repaired using the homologous sequence of the sister chromatid which serves as a template to repair the breaks.